{
  "term_id": "GO:0005634",
  "gene_symbol": "ZNF25",
  "gene": "UniProtKB:P17030",
  "term_label": "nucleus",
  "gene_name": "Zinc finger protein 25"
}